R8 cell fate commitment [GO:0007460] (biological process) Also known as: restriction of R8 fate Definition: The process in which the R8 photoreceptor commits to its cell fate. The R8 receptor contributes the central part of the rhabdomere in the basal parts of the ommatidium. References: PMID:3076112, PMID:3937883 Relationships: is a type of GO:0001752; is part of R8 cell differentiation [GO:0045465]